positive regulation of DNA recombination at centromere [GO:0061807] (biological process) Definition: Any process that activates or increases the frequency, rate or extent of DNA recombination at the centromere. Sources: GOC:dph, GOC:mah Also known as: positive regulation of centromeric recombination Relationships: is a type of positive regulation of DNA recombination [GO:0045911]; is a type of regulation of DNA recombination at centromere [GO:0061806]